{
  "term_id": "GO:0005789",
  "gene_symbol": "HACD3",
  "gene": "UniProtKB:Q9P035",
  "term_label": "endoplasmic reticulum membrane",
  "gene_name": "Very-long-chain (3R)-3-hydroxyacyl-CoA dehydratase 3"
}